regulation of gerfelin biosynthetic process [GO:1900686] (biological process) Definition: Any process that modulates the frequency, rate or extent of gerfelin biosynthetic process. Sources: GOC:TermGenie, GOC:di Subtypes: negative regulation of gerfelin biosynthetic process [GO:1900687], positive regulation of gerfelin biosynthetic process [GO:1900688] Also known as: regulation of gerfelin anabolism, regulation of gerfelin biosynthesis, regulation of gerfelin formation, regulation of gerfelin synthesis Relationships: is a type of regulation of ketone metabolic process [GO:0010565]; is a type of GO:0062012; is a type of regulation of secondary metabolite biosynthetic process [GO:1900376]; regulates GO:1900578